{
  "gene": "UniProtKB:P30530",
  "gene_symbol": "AXL",
  "term_label": "natural killer cell differentiation",
  "term_id": "GO:0001779",
  "gene_name": "Tyrosine-protein kinase receptor UFO"
}